{
  "term_label": "fructokinase activity",
  "gene_name": "Hexokinase-2",
  "term_id": "GO:0008865",
  "gene": "UniProtKB:P52789",
  "gene_symbol": "HK2"
}